{
  "gene_name": "Phosphatidylinositol 3,4,5-trisphosphate 3-phosphatase and dual-specificity protein phosphatase PTEN",
  "gene": "UniProtKB:P60484",
  "term_id": "GO:0043491",
  "term_label": "phosphatidylinositol 3-kinase/protein kinase B signal transduction",
  "gene_symbol": "PTEN"
}